interleukin-35 production [GO:0070753] (biological process) Regulation: regulated by regulation of interleukin-35 production [GO:0070754]; negatively regulated by negative regulation of interleukin-35 production [GO:0070755]; positively regulated by positive regulation of interleukin-35 production [GO:0070756] Relationships: is a type of cytokine production [GO:0001816] Definition: The appearance of interleukin-35 due to biosynthesis or secretion following a cellular stimulus, resulting in an increase in its intracellular or extracellular levels. Also known as: IL-35 production, interleukin-35 biosynthetic process, interleukin-35 secretion Sources: GOC:mah